{
  "gene": "UniProtKB:O75348",
  "gene_name": "V-type proton ATPase subunit G 1",
  "term_id": "GO:0030672",
  "term_label": "synaptic vesicle membrane",
  "gene_symbol": "ATP6V1G1"
}